{
  "gene_name": "A-kinase anchor protein 7 isoform gamma",
  "gene_symbol": "AKAP7",
  "gene": "UniProtKB:Q9P0M2",
  "term_label": "protein kinase A regulatory subunit binding",
  "term_id": "GO:0034237"
}